flight behavior [GO:0007629] (biological process) Relationships: is a type of adult locomotory behavior [GO:0008344] Also known as: flight behaviour Definition: The response to external or internal stimuli that results in the locomotory process of flight. Flight is the self-propelled movement of an organism through the air. Sources: GOC:jid, ISBN:0198606907